{
  "gene_name": "Dehydrodolichyl diphosphate synthase complex subunit NUS1",
  "gene": "UniProtKB:Q96E22",
  "term_label": "Unknown molecular function",
  "term_id": "UNKNOWN:0001",
  "gene_symbol": "NUS1"
}